{
  "gene": "UniProtKB:D6RA61",
  "gene_symbol": "USP17L22",
  "term_id": "GO:0031647",
  "term_label": "regulation of protein stability",
  "gene_name": "Ubiquitin carboxyl-terminal hydrolase 17-like protein 22"
}